aromatic (S)-hydroxynitrile lyase activity [GO:0052892] (molecular function) Definition: Catalysis of the reaction: an aromatic (S)-hydroxynitrile = an aromatic aldehyde + cyanide. Relationships: is a type of GO:0047606 Sources: RHEA:54660